{
  "gene_name": "Tubulin polymerization-promoting protein family member 2",
  "gene_symbol": "TPPP2",
  "term_label": "positive regulation of protein polymerization",
  "gene": "UniProtKB:P59282",
  "term_id": "GO:0032273"
}